{
  "term_label": "sperm head plasma membrane",
  "gene_symbol": "ADAM29",
  "gene": "UniProtKB:Q9UKF5",
  "term_id": "GO:1990913",
  "gene_name": "Disintegrin and metalloproteinase domain-containing protein 29"
}